{
  "gene_name": "WD repeat-containing protein 76",
  "gene": "UniProtKB:Q9H967",
  "gene_symbol": "WDR76",
  "term_label": "DNA binding",
  "term_id": "GO:0003677"
}